{
  "term_id": "GO:0005634",
  "term_label": "nucleus",
  "gene_symbol": "PRDM5",
  "gene": "UniProtKB:Q9NQX1",
  "gene_name": "PR domain zinc finger protein 5"
}